pheromone-dependent signal transduction involved in conjugation with cellular fusion [GO:0000750] (biological process) Regulation: regulated by regulation of pheromone-dependent signal transduction involved in conjugation with cellular fusion [GO:0010969]; positively regulated by GO:0090028; negatively regulated by negative regulation of pheromone-dependent signal transduction involved in conjugation with cellular fusion [GO:0090029] Definition: A signal transduction process resulting in the relay, amplification or dampening of a signal generated in response to pheromone exposure in organisms that undergo conjugation with cellular fusion. An example of this process is found in Saccharomyces cerevisiae. Sources: GOC:clt Relationships: is a type of signal transduction involved in positive regulation of conjugation with cellular fusion [GO:0032005]; is part of response to pheromone triggering conjugation with cellular fusion [GO:0000749] Also known as: transduction of mating signal